{
  "term_id": "GO:0005789",
  "term_label": "endoplasmic reticulum membrane",
  "gene_symbol": "SLC33A1",
  "gene_name": "Acetyl-coenzyme A transporter 1",
  "gene": "UniProtKB:O00400"
}